{
  "gene_symbol": "DCN",
  "term_label": "extracellular space",
  "term_id": "GO:0005615",
  "gene_name": "Decorin",
  "gene": "UniProtKB:P07585"
}